{
  "term_id": "GO:0006110",
  "term_label": "regulation of glycolytic process",
  "gene_symbol": "PRKAG2",
  "gene": "UniProtKB:Q9UGJ0",
  "gene_name": "5'-AMP-activated protein kinase subunit gamma-2"
}